{
  "gene_symbol": "CORO7",
  "term_label": "cell migration",
  "gene_name": "Coronin-7",
  "gene": "UniProtKB:P57737",
  "term_id": "GO:0016477"
}